{
  "term_label": "Unknown molecular function",
  "gene": "UniProtKB:Q86X40",
  "term_id": "UNKNOWN:0001",
  "gene_symbol": "LRRC28",
  "gene_name": "Leucine-rich repeat-containing protein 28"
}